xanthine transport [GO:0042906] (biological process) Also known as: xanthine transmembrane transport Definition: The directed movement of xanthine into, out of or within a cell, or between cells, by means of some agent such as a transporter or pore. Xanthine (2,6-dihydroxypurine) is a purine formed in the metabolic breakdown of guanine, but is not present in nucleic acids. Relationships: is a type of purine nucleobase transport [GO:0006863] Sources: GOC:jl